griseofulvin biosynthetic process [GO:0140878] (biological process) References: PMID:20534346, PMID:23978092 Relationships: is a type of mycotoxin biosynthetic process [GO:0043386]; is a type of GO:0090345 Also known as: griseofulvin anabolism, griseofulvin biosynthesis, griseofulvin formation, griseofulvin synthesis Definition: The chemical reactions and pathways resulting in the formation of griseofulvin, an important antifungal drug that has been in use for a long time for treating dermatophyte infections.